regulation of conidium formation [GO:0075306] (biological process) Sources: GOC:di, GOC:pamgo_curators Subtypes: positive regulation of conidium formation [GO:0075307], negative regulation of conidium formation [GO:0075308] Definition: Any process that modulates the frequency, rate or extent of conidium formation, a process of producing non-motile spores, called conidia, via mitotic asexual reproduction in higher fungi. Conidia are haploid cells genetically identical to their haploid parent. They are produced by conversion of hyphal elements, or are borne on sporogenous cells on or within specialized structures termed conidiophores, and participate in dispersal of the fungus. Relationships: is a type of regulation of asexual sporulation [GO:0034305]; is a type of regulation of cell development [GO:0060284]; regulates conidium formation [GO:0048315]